exocytic vesicle lumen [GO:0062246] (cellular component) Relationships: is_a GO:0098566; BFO_0000050 exocytic vesicle [GO:0070382] References: PMID:27384577 Definition: The volume enclosed by an exocytic vesicle.